{
  "term_label": "Unknown cellular component",
  "term_id": "UNKNOWN:0003",
  "gene_name": "Uncharacterized protein",
  "gene": "UniProtKB:A0A1B0GVB3",
  "gene_symbol": "LOC102725191"
}